{
  "gene_symbol": "NPS",
  "term_id": "GO:0032230",
  "term_label": "positive regulation of synaptic transmission, GABAergic",
  "gene": "UniProtKB:P0C0P6",
  "gene_name": "Neuropeptide S"
}